{
  "gene_name": "Casein kinase I isoform gamma-2",
  "term_label": "protein serine/threonine kinase activity",
  "term_id": "GO:0004674",
  "gene_symbol": "CSNK1G2",
  "gene": "UniProtKB:P78368"
}